negative regulation of B cell mediated immunity [GO:0002713] (BP) Sources: GOC:add Also known as: down regulation of B cell mediated immunity, down-regulation of B cell mediated immunity, downregulation of B cell mediated immunity, negative regulation of B lymphocyte mediated immunity, negative regulation of B-cell mediated immunity, negative regulation of B-lymphocyte mediated immunity, inhibition of B cell mediated immunity Subtypes: negative regulation of B cell antigen processing and presentation [GO:0002623], negative regulation of B cell cytokine production [GO:0002722], negative regulation of immunoglobulin mediated immune response [GO:0002890], negative regulation of peripheral B cell deletion [GO:0002909], negative regulation of peripheral B cell anergy [GO:0002918] Relationships: is a type of negative regulation of lymphocyte mediated immunity [GO:0002707]; is a type of regulation of B cell mediated immunity [GO:0002712]; is a type of negative regulation of adaptive immune response based on somatic recombination of immune receptors built from immunoglobulin superfamily domains [GO:0002823]; negatively regulates GO:0019724 Definition: Any process that stops, prevents, or reduces the frequency, rate, or extent of B cell mediated immunity.